determination of radial symmetry [GO:0009879] (BP) Also known as: determination of radial asymmetry Relationships: is a type of specification of symmetry [GO:0009799]; is part of radial pattern formation [GO:0009956] Sources: GOC:go_curators Definition: The establishment of an organism's body plan or a part of an organism such that it is symmetric around a central axis.